{
  "gene_name": "Rho-related GTP-binding protein RhoV",
  "term_label": "establishment of cell polarity",
  "gene_symbol": "RHOV",
  "term_id": "GO:0030010",
  "gene": "UniProtKB:Q96L33"
}